{
  "gene": "UniProtKB:P40259",
  "term_label": "B cell receptor signaling pathway",
  "gene_name": "B-cell antigen receptor complex-associated protein beta chain",
  "gene_symbol": "CD79B",
  "term_id": "GO:0050853"
}